{
  "gene": "UniProtKB:Q96SF7",
  "term_label": "DNA-binding transcription factor activity, RNA polymerase II-specific",
  "term_id": "GO:0000981",
  "gene_name": "T-box transcription factor TBX15",
  "gene_symbol": "TBX15"
}